{
  "term_label": "DNA-binding transcription factor activity, RNA polymerase II-specific",
  "gene_name": "Double homeobox protein 4-like protein 5",
  "gene": "UniProtKB:P0CJ88",
  "gene_symbol": "DUX4L5",
  "term_id": "GO:0000981"
}